{
  "gene_symbol": "ADAP1",
  "gene_name": "Arf-GAP with dual PH domain-containing protein 1",
  "term_label": "cytoplasm",
  "term_id": "GO:0005737",
  "gene": "UniProtKB:O75689"
}